{
  "gene_symbol": "MSH2",
  "gene": "UniProtKB:P43246",
  "term_id": "GO:0032301",
  "term_label": "MutSalpha complex",
  "gene_name": "DNA mismatch repair protein Msh2"
}